{
  "term_label": "RNA binding",
  "gene_symbol": "NELFCD",
  "gene": "UniProtKB:Q8IXH7",
  "gene_name": "Negative elongation factor C_D",
  "term_id": "GO:0003723"
}